regulation of antigen processing and presentation of peptide antigen via MHC class II [GO:0002586] (biological process) Definition: Any process that modulates the frequency, rate, or extent of antigen processing and presentation of peptide antigen via MHC class II. Relationships: is a type of GO:0002580; is a type of regulation of antigen processing and presentation of peptide antigen [GO:0002583]; regulates antigen processing and presentation of peptide antigen via MHC class II [GO:0002495] Sources: GOC:add Subtypes: negative regulation of antigen processing and presentation of peptide antigen via MHC class II [GO:0002587], positive regulation of antigen processing and presentation of peptide antigen via MHC class II [GO:0002588] Also known as: regulation of peptide antigen processing and presentation via MHC class II